{
  "term_id": "GO:0005829",
  "term_label": "cytosol",
  "gene_name": "Small ribosomal subunit protein eS1",
  "gene_symbol": "RPS3A",
  "gene": "UniProtKB:P61247"
}